regulation of protein targeting to vacuolar membrane [GO:1900483] (biological process) Subtypes: negative regulation of protein targeting to vacuolar membrane [GO:1900484], GO:1900485 Relationships: is a type of regulation of intracellular protein transport [GO:0033157]; is a type of regulation of protein targeting to membrane [GO:0090313]; is a type of regulation of vacuolar transport [GO:1903335]; is a type of regulation of protein localization to membrane [GO:1905475]; regulates protein targeting to vacuolar membrane [GO:0044395] Definition: Any process that modulates the frequency, rate or extent of protein targeting to vacuolar membrane. Sources: GOC:TermGenie